ribosomal large subunit binding [GO:0043023] (MF) Relationships: is a type of ribosome binding [GO:0043022] Definition: Binding to a large ribosomal subunit. Subtypes: mitochondrial large ribosomal subunit binding [GO:0140978] Sources: GOC:go_curators